symbiont-mediated suppression of host apoptosis [GO:0033668] (biological process) Definition: A process in which a symbiont inhibits or disrupts the normal execution of host apoptosis, leading to a decrease in the frequency, rate or extent of apoptosis in the host cell. The host is defined as the larger of the organisms involved in a symbiotic interaction. Also known as: down regulation by organism of host apoptotic programmed cell death, down-regulation by organism of host apoptotic programmed cell death, downregulation by organism of host apoptotic programmed cell death, inhibition by organism of host apoptotic programmed cell death, negative regulation by symbiont of host apoptosis, negative regulation by symbiont of host apoptotic process, suppression by symbiont of host apoptotic process, negative regulation by virus of host apoptosis, suppression by virus of host apoptosis Note: Note that term is to be used to annotate gene products in the symbiont. To annotate host gene products, consider the biological process term 'negative regulation of apoptosis ; GO:0043066'. Relationships: is a type of symbiont-mediated suppression of host programmed cell death [GO:0052041]; is_a GO:0052150 Sources: GOC:curators